{
  "term_id": "GO:0005615",
  "gene": "UniProtKB:O76061",
  "term_label": "extracellular space",
  "gene_name": "Stanniocalcin-2",
  "gene_symbol": "STC2"
}